{
  "term_label": "G protein-coupled receptor signaling pathway",
  "term_id": "GO:0007186",
  "gene": "UniProtKB:Q99677",
  "gene_name": "Lysophosphatidic acid receptor 4",
  "gene_symbol": "LPAR4"
}